DNA topological change [GO:0006265] (biological process) Relationships: is a type of DNA metabolic process [GO:0006259]; is_a DNA conformation change [GO:0071103] Sources: ISBN:071673706X, ISBN:0935702490 Also known as: DNA underwinding Definition: The process in which a transformation is induced in the topological structure of a double-stranded DNA helix, resulting in a change in linking number. Note: Note that the synonym 'DNA underwinding' should not be confused with 'DNA unwinding ; GO:0006268', which refers to DNA strand separation, and is a type of geometric change. GO:0006265 refers to alteration of the superhelical density of double-stranded DNA. Note that DNA topological change and DNA geometric change (GO:0032392) are distinct, but are usually coupled in vivo.